auxin biosynthetic process [GO:0009851] (biological process) Relationships: is a type of GO:0009850; is a type of hormone biosynthetic process [GO:0042446] Subtypes: indoleacetic acid biosynthetic process [GO:0009684], GO:0033474 Regulation: RO_0002211 by regulation of auxin biosynthetic process [GO:0010600]; positively regulated by positive regulation of auxin biosynthetic process [GO:0010601] Sources: GOC:lm, GOC:lr, ISBN:0122146743 Also known as: auxin anabolism, auxin biosynthesis, auxin formation, auxin synthesis Definition: The chemical reactions and pathways resulting in the formation of auxins, plant hormones that regulate aspects of plant growth.